fucosterol-epoxide lyase activity [GO:0047906] (molecular function) Sources: EC:4.1.2.33, RHEA:10884 Also known as: (24R,24'R)-fucosterol-epoxide acetaldehyde-lyase (desmosterol-forming), (24R,24'R)-fucosterol-epoxide acetaldehyde-lyase activity Definition: Catalysis of the reaction: (24R,24'R)-fucosterol epoxide = acetaldehyde + desmosterol. Relationships: is a type of GO:0016832